T cell mediated immune response to tumor cell [GO:0002424] (biological process) Relationships: is a type of immune response to tumor cell [GO:0002418]; is_a T cell mediated immunity [GO:0002456] Subtypes: T cell tolerance induction to tumor cell [GO:0002411], T cell mediated cytotoxicity directed against tumor cell target [GO:0002419] Regulation: regulated by regulation of T cell mediated immune response to tumor cell [GO:0002840]; negatively regulated by negative regulation of T cell mediated immune response to tumor cell [GO:0002841]; positively regulated by positive regulation of T cell mediated immune response to tumor cell [GO:0002842] References: PMID:16730260 Sources: GOC:add, ISBN:0781735149 Note: Note that this term includes tolerogenic responses to tumor cells mediated by responding T cells. Definition: An immune response mediated by a T cell triggered in response to the presence of a tumor cell.